{
  "term_id": "GO:0005886",
  "gene": "UniProtKB:Q9BT88",
  "gene_name": "Synaptotagmin-11",
  "term_label": "plasma membrane",
  "gene_symbol": "SYT11"
}